3-demethoxyubiquinone 3-hydroxylase (NADH) activity [GO:0160224] (molecular function) Definition: Catalysis of the reaction: a 5-methoxy-2-methyl-3-(all-trans-polyprenyl)benzoquinone + NADH + O2 = a 3-demethylubiquinone + NAD+ + H2O. Also known as: 5-methoxy-2-methyl-3-(all-trans-polyprenyl)benzoquinone,NADH:oxygen oxidoreductase (5-hydroxylating) activity Relationships: is a type of oxidoreductase activity, acting on paired donors, with incorporation or reduction of molecular oxygen, NAD(P)H as one donor, and incorporation of one atom of oxygen [GO:0016709] References: PMID:23445365, PMID:38425362 Sources: RHEA:81211